regulation of synaptic vesicle budding from presynaptic endocytic zone membrane [GO:0098694] (biological process) Definition: Any process that modulates the frequency, rate or extent of synaptic vesicle budding from presynaptic endocytic zone membrane. Relationships: is a type of regulation of organelle organization [GO:0033043]; regulates GO:0016185 Sources: GOC:dos